plant epidermis morphogenesis [GO:0090626] (biological process) Relationships: is a type of anatomical structure morphogenesis [GO:0009653]; is part of GO:0090558 Definition: The process in which the anatomical structures of the plant epidermis are generated and organized. Subtypes: GO:0010103 Sources: GOC:tb